{
  "gene": "UniProtKB:O95758",
  "gene_name": "Polypyrimidine tract-binding protein 3",
  "term_id": "GO:0003729",
  "term_label": "mRNA binding",
  "gene_symbol": "PTBP3"
}